{
  "term_id": "GO:0000981",
  "term_label": "DNA-binding transcription factor activity, RNA polymerase II-specific",
  "gene_symbol": "MSX1",
  "gene_name": "Homeobox protein MSX-1",
  "gene": "UniProtKB:P28360"
}